intracellular monoatomic anion homeostasis [GO:0030002] (biological process) Subtypes: intracellular chloride ion homeostasis [GO:0030644] Relationships: is a type of intracellular monoatomic ion homeostasis [GO:0006873]; is a type of GO:0055081 Definition: A homeostatic process involved in the maintenance of a steady state level of monoatomic anions within a cell. Monatomic anions (also called simple anions) are anions consisting of exactly one atom. Also known as: cellular anion homeostasis, cellular monoatomic anion homeostasis Sources: GOC:ceb, GOC:mah